chloroplast photosystem I binding [GO:0062067] (MF) Definition: Binding to a chloroplast photosystem I. References: PMID:17400553 Relationships: is a type of GO:0044877